{
  "gene_symbol": "ISG15",
  "gene_name": "Ubiquitin-like protein ISG15",
  "gene": "UniProtKB:P05161",
  "term_id": "GO:0019941",
  "term_label": "modification-dependent protein catabolic process"
}